{
  "gene_symbol": "FNTA",
  "term_label": "CAAX-protein geranylgeranyltransferase complex",
  "gene": "UniProtKB:P49354",
  "gene_name": "Protein farnesyltransferase_geranylgeranyltransferase type-1 subunit alpha",
  "term_id": "GO:0005953"
}